{
  "term_label": "Ras protein signal transduction",
  "gene_symbol": "RGL4",
  "term_id": "GO:0007265",
  "gene_name": "Ral-GDS-related protein",
  "gene": "UniProtKB:Q8IZJ4"
}